{
  "gene": "UniProtKB:P35711",
  "gene_name": "Transcription factor SOX-5",
  "gene_symbol": "SOX5",
  "term_id": "GO:0032332",
  "term_label": "positive regulation of chondrocyte differentiation"
}